regulation of generation of precursor metabolites and energy [GO:0043467] (BP) Sources: GOC:jl Relationships: is_a GO:0019222; regulates generation of precursor metabolites and energy [GO:0006091] Subtypes: regulation of glycolytic process [GO:0006110], regulation of photosynthesis, light reaction [GO:0042548], GO:0043456, regulation of cellular respiration [GO:0043457], regulation of fermentation [GO:0043465], regulation of glycogen metabolic process [GO:0070873], regulation of mitochondrial ATP synthesis coupled electron transport [GO:1905446] Definition: Any process that modulates the frequency, rate or extent of the chemical reactions and pathways resulting in the formation of precursor metabolites, substances from which energy is derived, and the processes involved in the liberation of energy from these substances.